{
  "gene": "UniProtKB:Q13546",
  "gene_name": "Receptor-interacting serine_threonine-protein kinase 1",
  "term_id": "GO:0004706",
  "gene_symbol": "RIPK1",
  "term_label": "JUN kinase kinase kinase activity"
}